methane biosynthetic process from methanethiol [GO:2001133] (BP) Regulation: regulated by regulation of methane biosynthetic process from methanethiol [GO:1900345]; negatively regulated by negative regulation of methane biosynthetic process from methanethiol [GO:1900346]; positively regulated by positive regulation of methane biosynthetic process from methanethiol [GO:1900347] Relationships: is_a sulfur compound metabolic process [GO:0006790]; is a type of methanogenesis [GO:0015948] Definition: The chemical reactions and pathways resulting in the formation of a methane from a methanethiol. Sources: GOC:mengo_curators